procambium histogenesis [GO:0010067] (biological process) Definition: The formation of the primary meristem or meristematic tissue that gives rise to the primary vascular tissue. Sources: GOC:tb, ISBN:0471245208 Relationships: is a type of primary meristem tissue development [GO:0010065]